{
  "term_id": "UNKNOWN:0002",
  "gene_name": "Voltage-dependent anion-selective channel protein 2",
  "term_label": "Unknown biological process",
  "gene_symbol": "VDAC2",
  "gene": "UniProtKB:P45880"
}